DNA synthesis involved in double-strand break repair via homologous recombination [GO:0043150] (biological process) Also known as: DNA synthesis during double-strand break repair via homologous recombination Sources: GOC:go_curators Relationships: is a type of DNA synthesis involved in DNA repair [GO:0000731]; is part of double-strand break repair via homologous recombination [GO:0000724] Definition: The synthesis of DNA that contributes to the process of double-strand break repair via homologous recombination.